{
  "term_id": "GO:0005856",
  "gene": "UniProtKB:Q16643",
  "gene_name": "Drebrin",
  "term_label": "cytoskeleton",
  "gene_symbol": "DBN1"
}